regulation of amoeboid sperm motility [GO:1905416] (biological process) Also known as: regulation of ameboid sperm motility, regulation of ameboid sperm movement, regulation of amoeboid sperm movement Sources: GOC:TermGenie, GOC:cilia, GOC:krc, GO_REF:0000058 Subtypes: negative regulation of amoeboid sperm motility [GO:1905417], positive regulation of amoeboid sperm motility [GO:1905418] Relationships: is a type of regulation of cell motility [GO:2000145]; is a type of regulation of reproductive process [GO:2000241]; regulates amoeboid sperm motility [GO:0097723] Definition: Any process that modulates the frequency, rate or extent of amoeboid sperm motility.